{
  "term_id": "GO:0008124",
  "gene_name": "Pterin-4-alpha-carbinolamine dehydratase 2",
  "gene": "UniProtKB:Q9H0N5",
  "term_label": "4-alpha-hydroxytetrahydrobiopterin dehydratase activity",
  "gene_symbol": "PCBD2"
}